regulation of cellular response to X-ray [GO:2000683] (biological process) Also known as: regulation of cellular response to X-ray radiation stimulus Relationships: is a type of regulation of response to stimulus [GO:0048583]; is a type of GO:0050794; regulates cellular response to X-ray [GO:0071481] Sources: GOC:obol Definition: Any process that modulates the frequency, rate or extent of cellular response to X-ray. Subtypes: negative regulation of cellular response to X-ray [GO:2000684], positive regulation of cellular response to X-ray [GO:2000685]